{
  "gene_name": "POTE ankyrin domain family member B3",
  "term_label": "Unknown biological process",
  "gene_symbol": "POTEB3",
  "gene": "UniProtKB:A0JP26",
  "term_id": "UNKNOWN:0002"
}